{
  "term_id": "GO:0097272",
  "term_label": "ammonium homeostasis",
  "gene_name": "Blood group Rh(CE) polypeptide",
  "gene": "UniProtKB:P18577",
  "gene_symbol": "RHCE"
}